{
  "gene_name": "Protocadherin-15",
  "gene_symbol": "PCDH15",
  "term_label": "cell adhesion",
  "gene": "UniProtKB:Q96QU1",
  "term_id": "GO:0007155"
}